{
  "gene_symbol": "ALOX15B",
  "term_label": "hepoxilin biosynthetic process",
  "gene_name": "Polyunsaturated fatty acid lipoxygenase ALOX15B",
  "gene": "UniProtKB:O15296",
  "term_id": "GO:0051122"
}